{
  "gene_symbol": "PLA2G4A",
  "term_label": "Golgi apparatus",
  "gene_name": "Cytosolic phospholipase A2",
  "term_id": "GO:0005794",
  "gene": "UniProtKB:P47712"
}